{
  "gene_symbol": "GPHA2",
  "term_id": "GO:0007166",
  "term_label": "cell surface receptor signaling pathway",
  "gene_name": "Glycoprotein hormone alpha-2",
  "gene": "UniProtKB:Q96T91"
}